{
  "term_label": "plasma membrane",
  "term_id": "GO:0005886",
  "gene": "UniProtKB:P31997",
  "gene_symbol": "CEACAM8",
  "gene_name": "Carcinoembryonic antigen-related cell adhesion molecule 8"
}